positive regulation of distal tip cell migration [GO:1903356] (biological process) Definition: Any process that activates or increases the frequency, rate or extent of distal tip cell migration. Relationships: is a type of GO:0030335; is a type of regulation of distal tip cell migration [GO:1903354]; positively regulates distal tip cell migration [GO:0097628] Also known as: up regulation of distal tip cell migration, up-regulation of distal tip cell migration, upregulation of distal tip cell migration, activation of distal tip cell migration References: PMID:24968003 Sources: GOC:TermGenie, GOC:mm2, GO_REF:0000058